{
  "gene": "UniProtKB:Q9BV68",
  "term_label": "ubiquitin protein ligase activity",
  "term_id": "GO:0061630",
  "gene_symbol": "RNF126",
  "gene_name": "E3 ubiquitin-protein ligase RNF126"
}